clathrin coating of Golgi vesicle, plasma membrane to endosome targeting [GO:0010785] (biological process) Definition: The addition of clathrin and adaptor proteins to Golgi membranes during the formation of transport vesicles that will move from the plasma membrane to the endosome, forming a vesicle coat. Sources: GOC:dph, GOC:tb Relationships: is a type of clathrin coating of Golgi vesicle [GO:0048202]; is part of GO:0048201